{
  "term_label": "lactate:proton symporter activity",
  "gene": "UniProtKB:P53985",
  "gene_symbol": "SLC16A1",
  "term_id": "GO:0015650",
  "gene_name": "Monocarboxylate transporter 1"
}